positive regulation of flagellated sperm motility involved in capacitation [GO:0060474] (biological process) Also known as: positive regulation of sperm motility involved in capacitation Definition: The process in which the controlled movement of a flagellated sperm cell is initiated as part of the process required for flagellated sperm to reach fertilization competence. Relationships: is a type of reproductive process [GO:0022414]; is a type of positive regulation of flagellated sperm motility [GO:1902093]; is part of GO:0048240 Sources: GOC:cilia, GOC:dph, GOC:krc